{
  "term_label": "nucleus",
  "term_id": "GO:0005634",
  "gene": "UniProtKB:Q00532",
  "gene_name": "Cyclin-dependent kinase-like 1",
  "gene_symbol": "CDKL1"
}